{
  "gene_name": "Pancreatic lipase-related protein 2",
  "gene": "UniProtKB:P54317",
  "gene_symbol": "PNLIPRP2",
  "term_label": "cholesterol homeostasis",
  "term_id": "GO:0042632"
}